{
  "gene_name": "Rhomboid-related protein 2",
  "gene": "UniProtKB:Q9NX52",
  "term_id": "UNKNOWN:0003",
  "gene_symbol": "RHBDL2",
  "term_label": "Unknown cellular component"
}